{
  "term_id": "GO:0015052",
  "term_label": "beta3-adrenergic receptor activity",
  "gene_name": "Beta-3 adrenergic receptor",
  "gene": "UniProtKB:P13945",
  "gene_symbol": "ADRB3"
}